sphingolipid biosynthetic process [GO:0030148] (BP) Also known as: sphingolipid anabolism, sphingolipid biosynthesis, sphingolipid formation, sphingolipid synthesis Subtypes: sphinganine-1-phosphate biosynthetic process [GO:0006669], GO:0006686, glycosphingolipid biosynthetic process [GO:0006688], ceramide biosynthetic process [GO:0046513], sphingoid biosynthetic process [GO:0046520], sphingolipid biosynthesis involved in endoplasmic reticulum membrane organization [GO:0090159], GO:1905373 Relationships: is a type of GO:0006665; is a type of membrane lipid biosynthetic process [GO:0046467] Definition: The chemical reactions and pathways resulting in the formation of sphingolipids, any of a class of lipids containing the long-chain amine diol sphingosine or a closely related base (a sphingoid). Sources: GOC:mah, ISBN:0198506732 Regulation: regulated by regulation of sphingolipid biosynthetic process [GO:0090153]; RO_0002213 by GO:0090154; negatively regulated by negative regulation of sphingolipid biosynthetic process [GO:0090155]